motor neuron axon guidance [GO:0008045] (biological process) Definition: The process in which the migration of an axon growth cone of a motor neuron is directed to a specific target site in response to a combination of attractive and repulsive cues. Sources: CL:0000100, GOC:pr, ISBN:0878932437 Also known as: motoneuron axon guidance, motor axon guidance, motor axon pathfinding Relationships: is_a GO:0007411 Subtypes: branchiomotor neuron axon guidance [GO:0021785] Regulation: regulated by regulation of motor neuron axon guidance [GO:1905812]; negatively regulated by negative regulation of motor neuron axon guidance [GO:1905813]; positively regulated by positive regulation of motor neuron axon guidance [GO:1905814]